{
  "gene": "UniProtKB:O43623",
  "gene_name": "Zinc finger protein SNAI2",
  "term_id": "GO:0006355",
  "term_label": "regulation of DNA-templated transcription",
  "gene_symbol": "SNAI2"
}